positive regulation of protein catabolic process in the vacuole [GO:1904352] (biological process) Also known as: up regulation of protein catabolic process in the vacuole, up-regulation of protein catabolic process in the vacuole, upregulation of protein catabolic process in the vacuole, activation of protein catabolic process in the vacuole, activation of vacuolar protein breakdown, activation of vacuolar protein catabolic process, activation of vacuolar protein catabolism, activation of vacuolar protein degradation, positive regulation of vacuolar protein breakdown, positive regulation of vacuolar protein catabolic process, positive regulation of vacuolar protein catabolism, positive regulation of vacuolar protein degradation, up regulation of vacuolar protein breakdown, up regulation of vacuolar protein catabolic process, up regulation of vacuolar protein catabolism, up regulation of vacuolar protein degradation, up-regulation of vacuolar protein breakdown, up-regulation of vacuolar protein catabolic process, up-regulation of vacuolar protein catabolism, up-regulation of vacuolar protein degradation, upregulation of vacuolar protein breakdown, upregulation of vacuolar protein catabolic process, upregulation of vacuolar protein catabolism, upregulation of vacuolar protein degradation Relationships: is a type of positive regulation of protein catabolic process [GO:0045732]; is a type of regulation of protein catabolic process in the vacuole [GO:1904350]; positively regulates protein catabolic process in the vacuole [GO:0007039] Definition: Any process that activates or increases the frequency, rate or extent of protein catabolic process in the vacuole. Subtypes: positive regulation of lysosomal protein catabolic process [GO:1905167] References: PMID:25635054 Sources: GOC:BHF, GOC:TermGenie, GOC:rl, GO_REF:0000058